{
  "gene_symbol": "SUGCT",
  "gene": "UniProtKB:Q9HAC7",
  "term_label": "mitochondrion",
  "gene_name": "Succinate--hydroxymethylglutarate CoA-transferase",
  "term_id": "GO:0005739"
}